{
  "term_label": "phosphatidylcholine metabolic process",
  "gene_symbol": "PLA2G2D",
  "gene": "UniProtKB:Q9UNK4",
  "term_id": "GO:0046470",
  "gene_name": "Group IID secretory phospholipase A2"
}